transposable element silencing by siRNA-mediated mRNA destabilization [GO:0141011] (biological process) Also known as: siRNA-mediated post-transcriptional retrotransposon silencing, siRNA-mediated retrotransposon silencing by mRNA destabilization References: PMID:36570931 Relationships: is a type of transposable element silencing by mRNA destabilization [GO:0141008] Definition: A transposable element silencing mechanism in which mRNAs transcribed from transposons are targeted for degradation by a siRNA.